methylmercury catabolic process [GO:0042193] (biological process) Definition: The chemical reactions and pathways resulting in the breakdown of methylmercury (MeHg+), a highly toxic organometal. Sources: GOC:ai Also known as: methylmercury breakdown, methylmercury catabolism, methylmercury degradation Relationships: is a type of catabolic process [GO:0009056]; is a type of organometal metabolic process [GO:0018942]